{
  "gene": "UniProtKB:A0A096LP55",
  "gene_symbol": "UQCRHL",
  "term_id": "UNKNOWN:0001",
  "gene_name": "Cytochrome b-c1 complex subunit 6-like, mitochondrial",
  "term_label": "Unknown molecular function"
}